{
  "term_id": "GO:0005886",
  "gene_symbol": "KCNK18",
  "term_label": "plasma membrane",
  "gene_name": "Potassium channel subfamily K member 18",
  "gene": "UniProtKB:Q7Z418"
}